{
  "term_id": "GO:0031012",
  "gene": "UniProtKB:Q9UKP5",
  "term_label": "extracellular matrix",
  "gene_name": "A disintegrin and metalloproteinase with thrombospondin motifs 6",
  "gene_symbol": "ADAMTS6"
}